{
  "gene_symbol": "STAT1",
  "gene": "UniProtKB:P42224",
  "term_id": "GO:0000981",
  "term_label": "DNA-binding transcription factor activity, RNA polymerase II-specific",
  "gene_name": "Signal transducer and activator of transcription 1-alpha_beta"
}